{
  "gene_symbol": "HSPA6",
  "gene": "UniProtKB:P17066",
  "gene_name": "Heat shock 70 kDa protein 6",
  "term_label": "cytoplasm",
  "term_id": "GO:0005737"
}